happens during [RO:0002092] (external) Relationships: subPropertyOf ends during [RO:0002093]